{
  "term_id": "UNKNOWN:0001",
  "gene": "UniProtKB:A1L4K1",
  "gene_symbol": "FSD2",
  "gene_name": "Fibronectin type III and SPRY domain-containing protein 2",
  "term_label": "Unknown molecular function"
}